determination of affect [GO:0050894] (biological process) Sources: GOC:ai, GOC:dph, ISBN:0721662544 Relationships: is a type of sensory processing [GO:0050893] Definition: Any process in which an emotional response is associated with a particular sensory stimulation.